{
  "gene_symbol": "CLTB",
  "gene": "UniProtKB:P09497",
  "gene_name": "Clathrin light chain B",
  "term_id": "GO:0030672",
  "term_label": "synaptic vesicle membrane"
}